{
  "term_id": "GO:0005737",
  "gene": "UniProtKB:P30613",
  "term_label": "cytoplasm",
  "gene_symbol": "PKLR",
  "gene_name": "Pyruvate kinase PKLR"
}